positive regulation of T cell mediated cytotoxicity directed against tumor cell target [GO:0002854] (biological process) Relationships: is a type of positive regulation of T cell mediated cytotoxicity [GO:0001916]; is a type of positive regulation of T cell mediated immune response to tumor cell [GO:0002842]; is a type of GO:0002852; positively regulates T cell mediated cytotoxicity directed against tumor cell target [GO:0002419] Also known as: up regulation of T cell mediated cytotoxicity directed against tumor cell target, up-regulation of T cell mediated cytotoxicity directed against tumor cell target, upregulation of T cell mediated cytotoxicity directed against tumor cell target, activation of T cell mediated cytotoxicity directed against tumor cell target, stimulation of T cell mediated cytotoxicity directed against tumor cell target Sources: GOC:add Definition: Any process that activates or increases the frequency, rate, or extent of T cell mediated cytotoxicity directed against a tumor cell target.